{
  "term_label": "cell projection",
  "gene": "UniProtKB:P48065",
  "gene_name": "Sodium- and chloride-dependent betaine transporter",
  "term_id": "GO:0042995",
  "gene_symbol": "SLC6A12"
}